{
  "gene_name": "ATPase family AAA domain-containing protein 5",
  "term_id": "GO:0061860",
  "term_label": "DNA clamp unloader activity",
  "gene": "UniProtKB:Q96QE3",
  "gene_symbol": "ATAD5"
}